{
  "gene_name": "Olfactory receptor 5M3",
  "term_id": "GO:0007608",
  "gene": "UniProtKB:Q8NGP4",
  "term_label": "sensory perception of smell",
  "gene_symbol": "OR5M3"
}